{
  "gene_name": "Putative olfactory receptor 10D4",
  "gene_symbol": "OR10D4P",
  "term_id": "GO:0050911",
  "term_label": "detection of chemical stimulus involved in sensory perception of smell",
  "gene": "UniProtKB:Q8NGN7"
}